positive regulation of vitamin E biosynthetic process [GO:1904966] (biological process) Definition: Any process that activates or increases the frequency, rate or extent of vitamin E biosynthetic process. Also known as: positive regulation of tocopherol biosynthesis, positive regulation of tocopherol biosynthetic process, positive regulation of vitamin E anabolism, positive regulation of vitamin E biosynthesis, positive regulation of vitamin E formation, positive regulation of vitamin E synthesis, up regulation of tocopherol biosynthesis, up regulation of tocopherol biosynthetic process, up regulation of vitamin E anabolism, up regulation of vitamin E biosynthesis, up regulation of vitamin E biosynthetic process, up regulation of vitamin E formation, up regulation of vitamin E synthesis, up-regulation of tocopherol biosynthesis, up-regulation of tocopherol biosynthetic process, up-regulation of vitamin E anabolism, up-regulation of vitamin E biosynthesis, up-regulation of vitamin E biosynthetic process, up-regulation of vitamin E formation, up-regulation of vitamin E synthesis, upregulation of tocopherol biosynthesis, upregulation of tocopherol biosynthetic process, upregulation of vitamin E anabolism, upregulation of vitamin E biosynthesis, upregulation of vitamin E biosynthetic process, upregulation of vitamin E formation, upregulation of vitamin E synthesis, activation of alpha-tocopherol biosynthesis, activation of alpha-tocopherol biosynthetic process, activation of tocopherol biosynthesis, activation of tocopherol biosynthetic process, activation of vitamin E anabolism, activation of vitamin E biosynthesis, activation of vitamin E biosynthetic process, activation of vitamin E formation, activation of vitamin E synthesis, positive regulation of alpha-tocopherol biosynthesis, positive regulation of alpha-tocopherol biosynthetic process, up regulation of alpha-tocopherol biosynthesis, up regulation of alpha-tocopherol biosynthetic process, up-regulation of alpha-tocopherol biosynthesis, up-regulation of alpha-tocopherol biosynthetic process, upregulation of alpha-tocopherol biosynthesis, upregulation of alpha-tocopherol biosynthetic process Relationships: is_a positive regulation of biosynthetic process [GO:0009891]; is a type of GO:0046136; is a type of regulation of vitamin E biosynthetic process [GO:1904965]; positively regulates vitamin E biosynthetic process [GO:0010189] References: PMID:20823244 Sources: GOC:TermGenie, GO_REF:0000058